phaseic acid biosynthetic process [GO:0010379] (biological process) Relationships: is a type of sesquiterpenoid biosynthetic process [GO:0016106]; is a type of apocarotenoid biosynthetic process [GO:0043289]; is a type of GO:0072330 Definition: The chemical reactions and pathways resulting in the formation of phaseic acid (PA), a catabolite of the plant hormone abscisic acid (ABA). Sources: MetaCyc:PWY-5271